electron transfer flavoprotein complex [GO:0045251] (cellular component) Definition: A protein complex facilitating the electron transfer from an acyl-CoA molecule to ubiquinone via its flavin adenine dinucleotide (FAD) cofactor. Usually contains an alpha and a beta subunit and the structural cofactor adenosine monophosphate (AMP). Part of a system that oxidizes an acyl-CoA molecule and reduces ubiquinone and other acceptors in the electron transport system. Also known as: ETF complex Sources: GOC:bhm, ISBN:0198506732 Relationships: is_a protein-containing complex [GO:0032991]; is part of cytoplasm [GO:0005737] Subtypes: mitochondrial electron transfer flavoprotein complex [GO:0017133], GO:0045247